positive regulation of interleukin-5 production [GO:0032754] (biological process) Definition: Any process that activates or increases the frequency, rate, or extent of interleukin-5 production. Also known as: positive regulation of IL-5 production, up regulation of interleukin-5 production, up-regulation of interleukin-5 production, upregulation of interleukin-5 production, activation of interleukin-5 production, positive regulation of interleukin-5 biosynthetic process, positive regulation of interleukin-5 secretion, stimulation of interleukin-5 production Relationships: is a type of positive regulation of cytokine production [GO:0001819]; is a type of regulation of interleukin-5 production [GO:0032674]; positively regulates interleukin-5 production [GO:0032634] Sources: GOC:mah